{
  "gene": "UniProtKB:Q15437",
  "gene_symbol": "SEC23B",
  "term_id": "GO:0030127",
  "term_label": "COPII vesicle coat",
  "gene_name": "Protein transport protein Sec23B"
}